artery development [GO:0060840] (biological process) Definition: The progression of the artery over time, from its initial formation to the mature structure. An artery is a blood vessel that carries blood away from the heart to a capillary bed. Sources: GOC:dph, GOC:sdb_2009, GOC:tb Relationships: is_a blood vessel development [GO:0001568] Subtypes: GO:0035904